{
  "term_label": "Unknown molecular function",
  "term_id": "UNKNOWN:0001",
  "gene": "UniProtKB:Q8NFP0",
  "gene_name": "Peroxisomal testis-specific protein 1",
  "gene_symbol": "PXT1"
}